negative regulation of protein folding [GO:1903333] (biological process) Definition: Any process that stops, prevents or reduces the frequency, rate or extent of protein folding. Sources: GOC:TermGenie, GOC:vw, GO_REF:0000058 Also known as: down regulation of protein folding, down-regulation of protein folding, downregulation of protein folding, down regulation of alpha-tubulin folding, down regulation of beta-tubulin folding, down regulation of chaperonin-mediated tubulin folding, down-regulation of alpha-tubulin folding, down-regulation of beta-tubulin folding, down-regulation of chaperonin-mediated tubulin folding, downregulation of alpha-tubulin folding, downregulation of beta-tubulin folding, downregulation of chaperonin-mediated tubulin folding, inhibition of alpha-tubulin folding, inhibition of beta-tubulin folding, inhibition of chaperonin-mediated tubulin folding, inhibition of protein folding, negative regulation of alpha-tubulin folding, negative regulation of beta-tubulin folding, negative regulation of chaperonin-mediated tubulin folding, down regulation of chaperone activity, down regulation of chaperonin ATPase activity, down regulation of co-chaperone activity, down regulation of co-chaperonin activity, down regulation of glycoprotein-specific chaperone activity, down regulation of non-chaperonin molecular chaperone ATPase activity, down regulation of protein complex assembly, multichaperone pathway, down-regulation of chaperone activity, down-regulation of chaperonin ATPase activity, down-regulation of co-chaperone activity, down-regulation of co-chaperonin activity, down-regulation of glycoprotein-specific chaperone activity, down-regulation of non-chaperonin molecular chaperone ATPase activity, down-regulation of protein complex assembly, multichaperone pathway, downregulation of chaperone activity, downregulation of chaperonin ATPase activity, downregulation of co-chaperone activity, downregulation of co-chaperonin activity, downregulation of glycoprotein-specific chaperone activity, downregulation of non-chaperonin molecular chaperone ATPase activity, downregulation of protein complex assembly, multichaperone pathway, inhibition of chaperone activity, inhibition of chaperonin ATPase activity, inhibition of co-chaperone activity, inhibition of co-chaperonin activity, inhibition of glycoprotein-specific chaperone activity, inhibition of non-chaperonin molecular chaperone ATPase activity, inhibition of protein complex assembly, multichaperone pathway, negative regulation of chaperone activity, negative regulation of chaperonin ATPase activity, negative regulation of co-chaperone activity, negative regulation of co-chaperonin activity, negative regulation of glycoprotein-specific chaperone activity, negative regulation of non-chaperonin molecular chaperone ATPase activity, negative regulation of protein complex assembly, multichaperone pathway Relationships: is a type of negative regulation of cellular process [GO:0048523]; is a type of regulation of protein folding [GO:1903332]; negatively regulates GO:0006457 Subtypes: negative regulation of protein refolding [GO:0061084]